5-amino-6-(5-phosphoribosylamino)uracil reductase activity [GO:0008703] (MF) Relationships: is a type of oxidoreductase activity, acting on the CH-OH group of donors, NAD or NADP as acceptor [GO:0016616] Sources: EC:1.1.1.193, RHEA:17845 Also known as: 5-amino-6-(5'-phosphoribosylamino)uracil reductase activity, 5-amino-6-(5-phosphoribitylamino)uracil:NADP+ 1'-oxidoreductase activity, aminodioxyphosphoribosylaminopyrimidine reductase activity Definition: Catalysis of the reaction: 5-amino-6-(5-phosphoribitylamino)uracil + NADP+ = 5-amino-6-(5-phosphoribosylamino)uracil + H+ + NADPH.